{
  "gene": "UniProtKB:Q8WXC3",
  "gene_symbol": "PYDC1",
  "term_label": "cytosol",
  "gene_name": "Pyrin domain-containing protein 1",
  "term_id": "GO:0005829"
}